positive regulation of cell division [GO:0051781] (biological process) Definition: Any process that activates or increases the frequency, rate or extent of cell division. Relationships: is a type of GO:0048522; is a type of regulation of cell division [GO:0051302]; positively regulates GO:0051301 Also known as: up regulation of cell division, up-regulation of cell division, upregulation of cell division, activation of cell division, stimulation of cell division Subtypes: positive regulation of cytokinesis [GO:0032467], positive regulation of asymmetric cell division [GO:0045770], positive regulation of cell budding [GO:0045782], positive regulation of somatic stem cell division [GO:1904677] Sources: GOC:ai